monoterpenoid catabolic process [GO:0016100] (biological process) Definition: The chemical reactions and pathways resulting in the breakdown of monoterpenoid compounds, terpenoids having a C10 skeleton. Sources: GOC:go_curators Also known as: monoterpenoid breakdown, monoterpenoid catabolism, monoterpenoid degradation Relationships: is a type of GO:0016098; is a type of terpenoid catabolic process [GO:0016115] Subtypes: GO:0019383, 6-hydroxycineole catabolic process [GO:0019639], geraniol catabolic process [GO:1903447]